{
  "gene_name": "Cyclin-dependent kinase 15",
  "gene": "UniProtKB:Q96Q40",
  "term_label": "cytosol",
  "term_id": "GO:0005829",
  "gene_symbol": "CDK15"
}